{
  "gene_name": "Immunoglobulin lambda variable 7-43",
  "gene_symbol": "IGLV7-43",
  "term_label": "immune response",
  "gene": "UniProtKB:P04211",
  "term_id": "GO:0006955"
}